{
  "gene": "UniProtKB:O95365",
  "gene_symbol": "ZBTB7A",
  "term_id": "GO:0006357",
  "gene_name": "Zinc finger and BTB domain-containing protein 7A",
  "term_label": "regulation of transcription by RNA polymerase II"
}